{
  "gene": "UniProtKB:Q12955",
  "term_label": "transmembrane transporter binding",
  "gene_name": "Ankyrin-3",
  "gene_symbol": "ANK3",
  "term_id": "GO:0044325"
}